{
  "gene_name": "Keratin, type II cytoskeletal 79",
  "gene_symbol": "KRT79",
  "term_id": "GO:0031424",
  "gene": "UniProtKB:Q5XKE5",
  "term_label": "keratinization"
}